enzyme-linked receptor protein signaling pathway [GO:0007167] (biological process) Definition: The series of molecular signals initiated by an extracellular ligand binding to a receptor on the surface of the target cell, where the receptor possesses catalytic activity or is closely associated with an enzyme such as a protein kinase, and ending with the regulation of a downstream cellular process, e.g. transcription. Sources: GOC:mah, GOC:signaling, ISBN:0815316194 Also known as: enzyme linked receptor protein signaling pathway, enzyme linked receptor protein signalling pathway Relationships: is a type of cell surface receptor signaling pathway [GO:0007166] Subtypes: receptor guanylyl cyclase signaling pathway [GO:0007168], cell surface receptor protein tyrosine kinase signaling pathway [GO:0007169], GO:0007178, cell surface receptor protein tyrosine phosphatase signaling pathway [GO:0007185], GO:0048861